{
  "term_id": "UNKNOWN:0001",
  "gene_name": "Tetraspanin-11",
  "term_label": "Unknown molecular function",
  "gene": "UniProtKB:A1L157",
  "gene_symbol": "TSPAN11"
}